{
  "term_id": "GO:0140284",
  "gene_name": "Motile sperm domain-containing protein 2",
  "term_label": "endoplasmic reticulum-endosome membrane contact site",
  "gene": "UniProtKB:Q8NHP6",
  "gene_symbol": "MOSPD2"
}